{
  "gene": "UniProtKB:O60486",
  "gene_symbol": "PLXNC1",
  "term_id": "GO:0005886",
  "gene_name": "Plexin-C1",
  "term_label": "plasma membrane"
}